{
  "term_id": "GO:0036126",
  "gene": "UniProtKB:Q658L1",
  "gene_symbol": "SAXO2",
  "term_label": "sperm flagellum",
  "gene_name": "Stabilizer of axonemal microtubules 2"
}